negative regulation of stomatal complex development [GO:2000122] (biological process) Definition: Any process that stops, prevents, or reduces the frequency, rate or extent of stomatal complex development. Relationships: is_a negative regulation of post-embryonic development [GO:0048581]; is a type of regulation of stomatal complex development [GO:2000038]; RO_0002212 stomatal complex development [GO:0010374] Sources: GOC:obol